{
  "gene_name": "Aquaporin-10",
  "gene": "UniProtKB:Q96PS8",
  "gene_symbol": "AQP10",
  "term_id": "GO:0016323",
  "term_label": "basolateral plasma membrane"
}